epithalamus development [GO:0021538] (biological process) Definition: The progression of the epithalamus over time from its initial formation until its mature state. The epithalamus is the small dorsomedial area of the thalamus including the habenular nuclei and associated fiber bundles, the pineal body, and the epithelial roof of the third ventricle. Relationships: is a type of anatomical structure development [GO:0048856]; is part of diencephalon development [GO:0021536] Sources: GOC:cls, GOC:dgh, GOC:dph, GOC:jid, GO_REF:0000021